{
  "gene": "UniProtKB:Q9HB40",
  "term_id": "UNKNOWN:0003",
  "term_label": "Unknown cellular component",
  "gene_symbol": "SCPEP1",
  "gene_name": "Retinoid-inducible serine carboxypeptidase"
}